{
  "gene_symbol": "FERMT1",
  "gene": "UniProtKB:Q9BQL6",
  "gene_name": "Fermitin family homolog 1",
  "term_label": "focal adhesion",
  "term_id": "GO:0005925"
}